{
  "term_label": "Unknown molecular function",
  "gene_name": "Tumor protein p53-inducible protein 13",
  "gene_symbol": "TP53I13",
  "term_id": "UNKNOWN:0001",
  "gene": "UniProtKB:Q8NBR0"
}